{
  "gene_name": "Homeobox protein Hox-C6",
  "term_label": "regulation of transcription by RNA polymerase II",
  "term_id": "GO:0006357",
  "gene": "UniProtKB:P09630",
  "gene_symbol": "HOXC6"
}